{
  "term_id": "GO:0019814",
  "term_label": "immunoglobulin complex",
  "gene_symbol": "IGKV3-11",
  "gene_name": "Immunoglobulin kappa variable 3-11",
  "gene": "UniProtKB:P04433"
}